minus-end directed microfilament motor activity [GO:0060001] (molecular function) Definition: A motor activity that generates movement along a microfilament towards the minus end, driven by ATP hydrolysis. The minus end of an actin filament is the end that does not preferentially add actin monomers. References: PMID:10519557 Sources: GOC:dph Also known as: minus-end directed actin-filament motor activity, pointed-end directed actin-filament motor activity, minus-end directed actin filament motor activity Relationships: is a type of GO:0000146